{
  "gene_name": "Speckle targeted PIP5K1A-regulated poly(A) polymerase",
  "term_label": "RNA 3'-end processing",
  "term_id": "GO:0031123",
  "gene_symbol": "TUT1",
  "gene": "UniProtKB:Q9H6E5"
}